{
  "gene_name": "Polyadenylate-binding protein 1",
  "term_label": "nucleus",
  "gene": "UniProtKB:P11940",
  "gene_symbol": "PABPC1",
  "term_id": "GO:0005634"
}